{
  "gene": "UniProtKB:O75888",
  "term_id": "GO:0030890",
  "term_label": "positive regulation of B cell proliferation",
  "gene_name": "Tumor necrosis factor ligand superfamily member 13",
  "gene_symbol": "TNFSF13"
}